protein import into peroxisome matrix [GO:0016558] (biological process) Definition: The import of proteins into the peroxisomal matrix. A peroxisome targeting signal (PTS) binds to a soluble receptor protein in the cytosol, and the resulting complex then binds to a receptor protein in the peroxisome membrane and is imported. The cargo protein is then released into the peroxisome matrix. References: PMID:11687502, PMID:11988772 Sources: ISBN:0716731363 Relationships: is a type of peroxisomal membrane transport [GO:0015919]; is a type of protein transmembrane import into intracellular organelle [GO:0044743]; is a type of GO:0072662; is_a establishment of protein localization to peroxisome [GO:0072663] Also known as: peroxisome matrix protein import, protein transport to peroxisome matrix